{
  "term_label": "Unknown molecular function",
  "term_id": "UNKNOWN:0001",
  "gene_name": "Chemokine-like factor",
  "gene": "UniProtKB:Q9UBR5",
  "gene_symbol": "CKLF"
}